{
  "gene_symbol": "POPDC3",
  "gene_name": "Popeye domain-containing protein 3",
  "term_label": "skeletal muscle tissue development",
  "term_id": "GO:0007519",
  "gene": "UniProtKB:Q9HBV1"
}